peptide histaminyltransferase activity [GO:0120299] (molecular function) Relationships: is a type of GO:0016410 References: PMID:23022564, PMID:23797785 Sources: GOC:sp Definition: Catalysis of the reaction: histamine + L-glutaminyl-[protein] = 5-histaminyl-L-glutamyl-[protein].